elongation of arista lateral [GO:0035016] (biological process) References: PMID:11404081 Sources: GOC:bf Relationships: is a type of developmental growth involved in morphogenesis [GO:0060560]; is part of antennal morphogenesis [GO:0048800] Definition: The increase in length of the aristal laterals. The arista is the terminal segment of the antenna and consists of a central core and a series of lateral extensions.